{
  "gene": "UniProtKB:Q96M69",
  "term_id": "GO:0005829",
  "gene_symbol": "LRGUK",
  "term_label": "cytosol",
  "gene_name": "Leucine-rich repeat and guanylate kinase domain-containing protein"
}